{
  "gene_name": "Laminin subunit alpha-3",
  "term_id": "UNKNOWN:0001",
  "gene_symbol": "LAMA3",
  "term_label": "Unknown molecular function",
  "gene": "UniProtKB:Q16787"
}